regulation of L-dopa biosynthetic process [GO:1903195] (biological process) Definition: Any process that modulates the frequency, rate or extent of L-dopa biosynthetic process. Subtypes: negative regulation of L-dopa biosynthetic process [GO:1903196], GO:1903197 Sources: GOC:PARL, GOC:TermGenie, GOC:bf, GO_REF:0000058 Relationships: is a type of GO:0062012; is a type of regulation of amino acid biosynthetic process [GO:2000282]; regulates L-dopa biosynthetic process [GO:1903185] Also known as: regulation of L-dopa anabolism, regulation of L-dopa biosynthesis, regulation of L-dopa formation, regulation of L-dopa synthesis